taurine biosynthetic process [GO:0042412] (biological process) Sources: GOC:jl, ISBN:0198600461 Also known as: taurine anabolism, taurine biosynthesis, taurine formation, taurine synthesis Relationships: is a type of GO:0019530; is a type of GO:0046305 Regulation: regulated by regulation of taurine biosynthetic process [GO:0062089]; positively regulated by positive regulation of taurine biosynthetic process [GO:0062090] Definition: The chemical reactions and pathways resulting in the formation of taurine (2-aminoethanesulfonic acid), a sulphur-containing amino acid derivative important in the metabolism of fats.